(R)-citramalate synthase activity [GO:0043714] (molecular function) References: PMID:9864346 Sources: GOC:jl, RHEA:19045 Also known as: citramalate synthase Definition: Catalysis of the reaction: pyruvate + acetyl-CoA + H2O = (R)-citramalate + CoA. Relationships: is a type of acyltransferase activity, transferring groups other than amino-acyl groups [GO:0016747]